{
  "gene_name": "Bromodomain-containing protein 1",
  "gene_symbol": "BRD1",
  "gene": "UniProtKB:O95696",
  "term_id": "GO:0005634",
  "term_label": "nucleus"
}